{
  "gene_symbol": "ZBP1",
  "term_label": "antiviral innate immune response",
  "term_id": "GO:0140374",
  "gene_name": "Z-DNA-binding protein 1",
  "gene": "UniProtKB:Q9H171"
}